negative regulation of cellular response to very-low-density lipoprotein particle stimulus [GO:1905888] (biological process) Definition: Any process that stops, prevents or reduces the frequency, rate or extent of cellular response to very-low-density lipoprotein particle stimulus. Also known as: down regulation of cellular response to VLDL particle stimulus, down regulation of cellular response to very-low-density lipoprotein particle stimulus, down-regulation of cellular response to VLDL particle stimulus, down-regulation of cellular response to very-low-density lipoprotein particle stimulus, downregulation of cellular response to VLDL particle stimulus, downregulation of cellular response to very-low-density lipoprotein particle stimulus, negative regulation of cellular response to VLDL particle stimulus, inhibition of cellular response to VLDL particle stimulus, inhibition of cellular response to very-low-density lipoprotein particle stimulus Relationships: is_a negative regulation of cellular process [GO:0048523]; is a type of negative regulation of response to stimulus [GO:0048585]; is a type of regulation of cellular response to very-low-density lipoprotein particle stimulus [GO:1905890]; negatively regulates GO:0090731 References: PMID:7592957 Sources: GOC:TermGenie, GOC:aruk, GOC:bc, GO_REF:0000058